{
  "term_id": "UNKNOWN:0002",
  "gene": "UniProtKB:Q5JU69",
  "gene_name": "Torsin-2A",
  "gene_symbol": "TOR2A",
  "term_label": "Unknown biological process"
}